{
  "term_label": "protein kinase activity",
  "gene_name": "Mitotic checkpoint serine_threonine-protein kinase BUB1 beta",
  "gene_symbol": "BUB1B",
  "term_id": "GO:0004672",
  "gene": "UniProtKB:O60566"
}